{
  "gene_symbol": "KATNAL1",
  "gene": "UniProtKB:Q9BW62",
  "gene_name": "Katanin p60 ATPase-containing subunit A-like 1",
  "term_id": "GO:0016887",
  "term_label": "ATP hydrolysis activity"
}